{
  "term_label": "kininogen binding",
  "term_id": "GO:0030984",
  "gene": "UniProtKB:Q07021",
  "gene_symbol": "C1QBP",
  "gene_name": "Complement component 1 Q subcomponent-binding protein, mitochondrial"
}